{
  "gene_name": "Non-histone chromosomal protein HMG-17",
  "term_id": "GO:0003682",
  "gene_symbol": "HMGN2",
  "gene": "UniProtKB:P05204",
  "term_label": "chromatin binding"
}